{
  "gene_name": "Cytochrome c oxidase subunit 5B, mitochondrial",
  "gene_symbol": "COX5B",
  "term_label": "mitochondrial electron transport, cytochrome c to oxygen",
  "term_id": "GO:0006123",
  "gene": "UniProtKB:P10606"
}